{
  "gene": "UniProtKB:Q9BV94",
  "term_label": "endoplasmic reticulum",
  "gene_symbol": "EDEM2",
  "term_id": "GO:0005783",
  "gene_name": "ER degradation-enhancing alpha-mannosidase-like protein 2"
}